{
  "term_id": "UNKNOWN:0003",
  "gene": "UniProtKB:Q9NS26",
  "gene_name": "Sperm protein associated with the nucleus on the X chromosome A",
  "term_label": "Unknown cellular component",
  "gene_symbol": "SPANXA2"
}